positive regulation of maternal process involved in parturition [GO:1904303] (biological process) Relationships: is a type of positive regulation of multicellular organismal process [GO:0051240]; is_a regulation of maternal process involved in parturition [GO:1904301]; is a type of positive regulation of reproductive process [GO:2000243]; positively regulates maternal process involved in parturition [GO:0060137] Also known as: up regulation of maternal process involved in parturition, up-regulation of maternal process involved in parturition, upregulation of maternal process involved in parturition, activation of maternal process involved in parturition Definition: Any process that activates or increases the frequency, rate or extent of maternal process involved in parturition. References: PMID:1849751 Sources: GOC:TermGenie, GO_REF:0000058